{
  "term_label": "extracellular space",
  "gene_name": "Serpin A12",
  "term_id": "GO:0005615",
  "gene_symbol": "SERPINA12",
  "gene": "UniProtKB:Q8IW75"
}